{
  "gene_symbol": "PARL",
  "gene": "UniProtKB:Q9H300",
  "term_label": "mitochondrion",
  "gene_name": "Presenilin-associated rhomboid-like protein, mitochondrial",
  "term_id": "GO:0005739"
}